{
  "gene_name": "Bcl2-associated agonist of cell death",
  "term_label": "cysteine-type endopeptidase activator activity",
  "gene_symbol": "BAD",
  "gene": "UniProtKB:Q92934",
  "term_id": "GO:0140608"
}